{
  "gene": "UniProtKB:A0A087WSY6",
  "term_id": "GO:0006955",
  "gene_name": "Immunoglobulin kappa variable 3D-15",
  "term_label": "immune response",
  "gene_symbol": "IGKV3D-15"
}